{
  "gene_name": "V-type proton ATPase subunit F",
  "term_label": "membrane",
  "gene": "UniProtKB:Q16864",
  "gene_symbol": "ATP6V1F",
  "term_id": "GO:0016020"
}